{
  "term_id": "UNKNOWN:0001",
  "gene": "UniProtKB:A0A8V8TNB9",
  "gene_name": "Uncharacterized protein",
  "gene_symbol": "A0A8V8TNB9",
  "term_label": "Unknown molecular function"
}